{
  "gene_symbol": "RBMY1A1",
  "term_label": "spliceosomal complex",
  "term_id": "GO:0005681",
  "gene": "UniProtKB:P0DJD3",
  "gene_name": "RNA-binding motif protein, Y chromosome, family 1 member A1"
}